positive regulation of mesodermal cell fate specification [GO:0048337] (biological process) Definition: Any process that activates or increases the frequency, rate or extent of mesoderm cell fate specification. Subtypes: GO:0048330, positive regulation of paraxial mesodermal cell fate specification [GO:0048350], positive regulation of lateral mesodermal cell fate specification [GO:0048379], positive regulation of intermediate mesodermal cell fate specification [GO:0048400] Relationships: is_a positive regulation of cell fate specification [GO:0042660]; is a type of regulation of mesodermal cell fate specification [GO:0042661]; is a type of positive regulation of mesodermal cell differentiation [GO:1905772]; positively regulates mesodermal cell fate specification [GO:0007501] Also known as: up regulation of mesodermal cell fate specification, up-regulation of mesodermal cell fate specification, upregulation of mesodermal cell fate specification, activation of mesodermal cell fate specification, stimulation of mesodermal cell fate specification Sources: GOC:dgh